{
  "gene_symbol": "GABRG1",
  "term_label": "inhibitory synapse assembly",
  "term_id": "GO:1904862",
  "gene_name": "Gamma-aminobutyric acid receptor subunit gamma-1",
  "gene": "UniProtKB:Q8N1C3"
}